{
  "gene": "UniProtKB:P43359",
  "gene_symbol": "MAGEA5P",
  "gene_name": "Putative melanoma-associated antigen 5P",
  "term_label": "Unknown biological process",
  "term_id": "UNKNOWN:0002"
}